{
  "gene_name": "Speedy protein E12",
  "term_id": "GO:0019901",
  "gene": "UniProtKB:P0DUX1",
  "gene_symbol": "SPDYE12",
  "term_label": "protein kinase binding"
}